regulation of organ growth [GO:0046620] (biological process) Definition: Any process that modulates the frequency, rate or extent of growth of an organ of an organism. Sources: GOC:bf, GOC:tb Relationships: is a type of regulation of developmental growth [GO:0048638]; is a type of regulation of multicellular organismal process [GO:0051239]; regulates organ growth [GO:0035265] Subtypes: negative regulation of organ growth [GO:0046621], positive regulation of organ growth [GO:0046622], regulation of heart growth [GO:0060420]